calcium channel regulator activity [GO:0005246] (molecular function) Definition: Modulates the activity of a calcium channel. Subtypes: calcium channel inhibitor activity [GO:0019855] Sources: GOC:mah Relationships: is a type of ion channel regulator activity [GO:0099106]; regulates GO:0005262